{
  "term_id": "GO:0005634",
  "gene_symbol": "CDAN1",
  "gene_name": "Codanin-1",
  "term_label": "nucleus",
  "gene": "UniProtKB:Q8IWY9"
}